{
  "gene_name": "Kinesin-like protein KIF2C",
  "gene_symbol": "KIF2C",
  "gene": "UniProtKB:Q99661",
  "term_label": "centrosome",
  "term_id": "GO:0005813"
}